{
  "term_label": "Unknown cellular component",
  "gene_symbol": "LRRFIP1",
  "gene": "UniProtKB:Q32MZ4",
  "gene_name": "Leucine-rich repeat flightless-interacting protein 1",
  "term_id": "UNKNOWN:0003"
}